{
  "gene_name": "Myozenin-1",
  "term_label": "actin cytoskeleton",
  "gene": "UniProtKB:Q9NP98",
  "gene_symbol": "MYOZ1",
  "term_id": "GO:0015629"
}